psychomotor behavior [GO:0036343] (BP) Definition: The specific behavior of an organism that combines cognitive functions and physical movement. For example, driving a car, throwing a ball, or playing a musical instrument. Relationships: is a type of motor behavior [GO:0061744] References: PMID:17159989 Sources: GOC:nhn, GOC:pr, Wikipedia:Psychomotor_learning